{
  "term_label": "Unknown molecular function",
  "gene": "UniProtKB:Q13884",
  "gene_name": "Beta-1-syntrophin",
  "term_id": "UNKNOWN:0001",
  "gene_symbol": "SNTB1"
}